{
  "gene": "UniProtKB:Q14416",
  "gene_name": "Metabotropic glutamate receptor 2",
  "term_id": "GO:0007216",
  "term_label": "G protein-coupled glutamate receptor signaling pathway",
  "gene_symbol": "GRM2"
}